{
  "gene_symbol": "GATM",
  "term_label": "glycine amidinotransferase activity",
  "gene_name": "Glycine amidinotransferase, mitochondrial",
  "gene": "UniProtKB:P50440",
  "term_id": "GO:0015068"
}